{
  "term_id": "GO:0006493",
  "term_label": "protein O-linked glycosylation",
  "gene": "UniProtKB:Q9UNA3",
  "gene_name": "Alpha-1,4-N-acetylglucosaminyltransferase",
  "gene_symbol": "A4GNT"
}